{
  "term_id": "GO:0070681",
  "gene_name": "Glutamyl-tRNA(Gln) amidotransferase subunit B, mitochondrial",
  "term_label": "glutaminyl-tRNAGln biosynthesis via transamidation",
  "gene_symbol": "GATB",
  "gene": "UniProtKB:O75879"
}